{
  "term_label": "Unknown molecular function",
  "gene": "UniProtKB:P63128",
  "gene_name": "Endogenous retrovirus group K member 9 Pol protein",
  "gene_symbol": "ERVK-9",
  "term_id": "UNKNOWN:0001"
}